{
  "gene_symbol": "LAT",
  "gene_name": "Linker for activation of T-cells family member 1",
  "gene": "UniProtKB:O43561",
  "term_label": "signaling receptor complex adaptor activity",
  "term_id": "GO:0030159"
}